{
  "term_label": "maturation of SSU-rRNA from tricistronic rRNA transcript (SSU-rRNA, 5.8S rRNA, LSU-rRNA)",
  "gene": "UniProtKB:Q8IY37",
  "term_id": "GO:0000462",
  "gene_symbol": "DHX37",
  "gene_name": "Probable ATP-dependent RNA helicase DHX37"
}